{
  "gene_symbol": "SPINK2",
  "term_id": "GO:0001669",
  "gene": "UniProtKB:P20155",
  "gene_name": "Serine protease inhibitor Kazal-type 2",
  "term_label": "acrosomal vesicle"
}